{
  "term_id": "GO:0022008",
  "gene": "UniProtKB:P61328",
  "gene_symbol": "FGF12",
  "gene_name": "Fibroblast growth factor 12",
  "term_label": "neurogenesis"
}